{
  "gene_symbol": "COMMD9",
  "gene_name": "COMM domain-containing protein 9",
  "term_id": "UNKNOWN:0002",
  "term_label": "Unknown biological process",
  "gene": "UniProtKB:Q9P000"
}